{
  "gene_name": "HMG box transcription factor BBX",
  "gene_symbol": "BBX",
  "term_label": "RNA polymerase II transcription regulatory region sequence-specific DNA binding",
  "term_id": "GO:0000977",
  "gene": "UniProtKB:Q8WY36"
}